positive regulation of lipid storage [GO:0010884] (biological process) Sources: GOC:BHF, GOC:dph, GOC:tb Definition: Any process that increases the rate, frequency or extent of lipid storage. Lipid storage is the accumulation and maintenance in cells or tissues of lipids, compounds soluble in organic solvents but insoluble or sparingly soluble in aqueous solvents. Lipid reserves can be accumulated during early developmental stages for mobilization and utilization at later stages of development. Relationships: is_a regulation of lipid storage [GO:0010883]; is a type of positive regulation of cellular process [GO:0048522]; is a type of positive regulation of lipid localization [GO:1905954]; positively regulates lipid storage [GO:0019915] Subtypes: positive regulation of cholesterol storage [GO:0010886], positive regulation of triglyceride storage [GO:0010890] Also known as: positive regulation of lipid sequestration